{
  "term_id": "GO:0012505",
  "gene_symbol": "CYB5D2",
  "gene": "UniProtKB:Q8WUJ1",
  "term_label": "endomembrane system",
  "gene_name": "Neuferricin"
}